peptidyl-lysine demalonylation [GO:0036047] (biological process) Definition: The process of removing a malonyl group (CO-CH2-CO) from an malonylated lysine residue in a peptide or protein. References: PMID:22076378 Sources: GOC:sp Relationships: is a type of peptidyl-lysine modification [GO:0018205]; is a type of GO:0036046